{
  "term_label": "inflammatory response",
  "gene": "UniProtKB:Q8WWZ1",
  "gene_symbol": "IL1F10",
  "term_id": "GO:0006954",
  "gene_name": "Interleukin-1 family member 10"
}